regulation of protein autophosphorylation [GO:0031952] (biological process) Sources: GOC:mah Also known as: regulation of protein amino acid autophosphorylation Definition: Any process that modulates the frequency, rate or extent of addition of the phosphorylation by a protein of one or more of its own residues. Subtypes: negative regulation of protein autophosphorylation [GO:0031953], positive regulation of protein autophosphorylation [GO:0031954], regulation of peptidyl-tyrosine autophosphorylation [GO:1900084] Relationships: is a type of regulation of protein phosphorylation [GO:0001932]; has part regulation of protein kinase activity [GO:0045859]; RO_0002211 protein autophosphorylation [GO:0046777]